{
  "gene_name": "Putative inactive neutral ceramidase B",
  "term_id": "UNKNOWN:0003",
  "gene": "UniProtKB:P0C7U1",
  "gene_symbol": "ASAH2B",
  "term_label": "Unknown cellular component"
}